{
  "term_label": "alpha-amylase activity",
  "gene_symbol": "AMY1C",
  "gene_name": "Alpha-amylase 1C",
  "term_id": "GO:0004556",
  "gene": "UniProtKB:P0DTE8"
}